actin filament bundle of filopodium [GO:0098861] (cellular component) References: PMID:12566431 Relationships: is a type of actin filament bundle of actin-based cell projection [GO:0098859]; BFO_0000050 filopodium [GO:0030175] Definition: A parallel bundle of actin filaments that is part of filopodium. Filaments are oriented such that the plus (barbed) ends are at the tip of the protrusion, capped by a tip complex.